{
  "gene_name": "APC membrane recruitment protein 1",
  "gene_symbol": "AMER1",
  "term_id": "GO:0005886",
  "gene": "UniProtKB:Q5JTC6",
  "term_label": "plasma membrane"
}